{
  "term_id": "GO:0005815",
  "gene_symbol": "STIL",
  "gene": "UniProtKB:Q15468",
  "gene_name": "SCL-interrupting locus protein",
  "term_label": "microtubule organizing center"
}